{
  "gene_symbol": "ZBTB1",
  "term_id": "GO:0000978",
  "term_label": "RNA polymerase II cis-regulatory region sequence-specific DNA binding",
  "gene_name": "Zinc finger and BTB domain-containing protein 1",
  "gene": "UniProtKB:Q9Y2K1"
}